{
  "term_id": "GO:0042981",
  "gene_symbol": "TP63",
  "term_label": "regulation of apoptotic process",
  "gene_name": "Tumor protein 63",
  "gene": "UniProtKB:Q9H3D4"
}